{
  "gene": "UniProtKB:Q8IZH2",
  "gene_symbol": "XRN1",
  "term_id": "GO:0000956",
  "gene_name": "5'-3' exoribonuclease 1",
  "term_label": "nuclear-transcribed mRNA catabolic process"
}